cysteine sulfinate desulfinase activity [GO:0008826] (molecular function) Sources: RHEA:28278 Relationships: is a type of carbon-sulfur lyase activity [GO:0016846] Also known as: cysteine sulphinate desulphinase activity Definition: Catalysis of the reaction: 3-sulfinoalanine = L-alanine + sulfite.